indolelactate dehydrogenase (NAD+) activity [GO:0047722] (molecular function) Relationships: is a type of oxidoreductase activity, acting on the CH-OH group of donors, NAD or NADP as acceptor [GO:0016616] Also known as: indole-3-lactate dehydrogenase activity, (indol-3-yl)lactate:NAD+ oxidoreductase activity, indolelactate:NAD+ oxidoreductase activity Sources: RHEA:20133 Definition: Catalysis of the reaction: 3-(indol-3-yl)lactate + NAD+ = 3-(indol-3-yl)pyruvate + H+ + NADH.